{
  "gene": "UniProtKB:P49238",
  "term_label": "C-C chemokine binding",
  "term_id": "GO:0019957",
  "gene_symbol": "CX3CR1",
  "gene_name": "CX3C chemokine receptor 1"
}